{
  "gene": "UniProtKB:P59044",
  "term_id": "GO:0005000",
  "term_label": "vasopressin receptor activity",
  "gene_symbol": "NLRP6",
  "gene_name": "NACHT, LRR and PYD domains-containing protein 6"
}